{
  "term_label": "bicarbonate transport",
  "gene_name": "Electroneutral sodium bicarbonate exchanger 1",
  "gene_symbol": "SLC4A8",
  "gene": "UniProtKB:Q2Y0W8",
  "term_id": "GO:0015701"
}